positive regulation of branching involved in lung morphogenesis [GO:0061047] (biological process) Definition: Any process that increases the rate, frequency, or extent of the process in which a highly ordered sequence of patterning events generates the branched structures of the lung, consisting of reiterated combinations of bud outgrowth, elongation, and dichotomous subdivision of terminal units. Subtypes: GO:0060504 Sources: GOC:dph, GOC:yaf Relationships: is a type of positive regulation of multicellular organismal process [GO:0051240]; is_a regulation of branching involved in lung morphogenesis [GO:0061046]; is_a positive regulation of morphogenesis of an epithelium [GO:1905332]; positively regulates epithelial tube branching involved in lung morphogenesis [GO:0060441]